{
  "term_label": "microtubule cytoskeleton",
  "gene": "UniProtKB:A6PVC2",
  "term_id": "GO:0015630",
  "gene_name": "Protein monoglycylase TTLL8",
  "gene_symbol": "TTLL8"
}